{
  "term_label": "ribonucleoprotein granule",
  "term_id": "GO:0035770",
  "gene": "UniProtKB:Q7L8L6",
  "gene_name": "FAST kinase domain-containing protein 5, mitochondrial",
  "gene_symbol": "FASTKD5"
}